{
  "gene": "UniProtKB:Q96C92",
  "gene_name": "Endosome-associated-trafficking regulator 1",
  "term_label": "Unknown molecular function",
  "gene_symbol": "ENTR1",
  "term_id": "UNKNOWN:0001"
}